hexose phosphate transport [GO:0015712] (biological process) Definition: The directed movement of hexose phosphate into, out of or within a cell, or between cells, by means of some agent such as a transporter or pore. Sources: GOC:krc Relationships: is a type of organophosphate ester transport [GO:0015748]; is a type of GO:1901264 Subtypes: glucose-6-phosphate transport [GO:0015760]